{
  "gene_symbol": "RNF228",
  "term_label": "protein ubiquitination",
  "gene_name": "RING-type domain-containing protein",
  "term_id": "GO:0016567",
  "gene": "UniProtKB:A0A7I2V3R4"
}